{
  "gene_symbol": "CEP76",
  "gene_name": "Centrosomal protein of 76 kDa",
  "gene": "UniProtKB:Q8TAP6",
  "term_id": "GO:0046599",
  "term_label": "regulation of centriole replication"
}